oxoglutarate dehydrogenase complex [GO:0045252] (cellular component) Note: The catalytic activities of the individual components of this complex are represented by the molecular function terms 'oxoglutarate dehydrogenase (succinyl-transferring) activity ; GO:0004591' (E1), 'dihydrolipoyllysine-residue succinyltransferase activity ; GO:0004149' (E2), and 'dihydrolipoyl dehydrogenase activity ; GO:0004148' (E3). Relationships: is a type of GO:0045239; is a type of alpha-ketoacid dehydrogenase complex [GO:0045240]; is a type of transferase complex [GO:1990234] References: PMID:10672230 Also known as: KGDHC, alpha-ketoglutarate dehydrogenase complex, dihydrolipoamide S-succinyltransferase complex Definition: A multi-enzyme complex that catalyzes the oxidative decarboxylation of alpha-ketoglutarate (also known as 2-oxoglutarate) to form succinyl-CoA. The complex comprises multiple copies of three enzymes referred to as E1, E2 and E3: oxoglutarate dehydrogenase (lipoamide) (E1), dihydrolipoamide S-succinyltransferase (E2) and dihydrolipoamide dehydrogenase (E3). Additional proteins may also be present.